{
  "gene": "UniProtKB:P30153",
  "term_label": "protein phosphatase regulator activity",
  "gene_symbol": "PPP2R1A",
  "term_id": "GO:0019888",
  "gene_name": "Serine_threonine-protein phosphatase 2A 65 kDa regulatory subunit A alpha isoform"
}